{
  "term_id": "GO:0005886",
  "gene_name": "Cell adhesion molecule DSCAML1",
  "term_label": "plasma membrane",
  "gene_symbol": "DSCAML1",
  "gene": "UniProtKB:Q8TD84"
}